{
  "gene": "UniProtKB:Q8IYX7",
  "gene_name": "Stabilizer of axonemal microtubules 1",
  "term_id": "GO:0005814",
  "gene_symbol": "SAXO1",
  "term_label": "centriole"
}